neurofilament bundle assembly [GO:0033693] (biological process) Definition: The assembly of neurofilaments into bundles, in which the filaments are longitudinally oriented, with numerous crossbridges between them. Neurofilament bundles may be cross-linked to each other, to membrane-bounded organelles or other cytoskeletal structures such as microtubules. References: PMID:11034913, PMID:11264295 Also known as: NF bundle assembly Relationships: is a type of GO:0045110